{
  "gene": "UniProtKB:Q9BYH1",
  "term_id": "UNKNOWN:0001",
  "gene_symbol": "SEZ6L",
  "gene_name": "Seizure 6-like protein",
  "term_label": "Unknown molecular function"
}